{
  "gene": "UniProtKB:P08709",
  "term_label": "extracellular space",
  "gene_symbol": "F7",
  "term_id": "GO:0005615",
  "gene_name": "Coagulation factor VII"
}